{
  "term_label": "purine-rich negative regulatory element binding",
  "term_id": "GO:0032422",
  "gene_name": "Transcriptional activator protein Pur-beta",
  "gene_symbol": "PURB",
  "gene": "UniProtKB:Q96QR8"
}